{
  "gene_symbol": "HPSE2",
  "term_id": "GO:0030198",
  "gene": "UniProtKB:Q8WWQ2",
  "gene_name": "Inactive heparanase-2",
  "term_label": "extracellular matrix organization"
}